positive regulation of MAPK cascade [GO:0043410] (biological process) Subtypes: GO:0032874, positive regulation of MAP kinase activity [GO:0043406], positive regulation of JNK cascade [GO:0046330], positive regulation of pheromone response MAPK cascade [GO:0062038], positive regulation of ERK1 and ERK2 cascade [GO:0070374], positive regulation of ERK5 cascade [GO:0070378], positive regulation of MAPKKK cascade by fibroblast growth factor receptor signaling pathway [GO:0090080], positive regulation of p38MAPK cascade [GO:1900745] Sources: GOC:go_curators Also known as: positive regulation of MAP kinase cascade, positive regulation of MAP kinase kinase kinase cascade, positive regulation of MAPKKK cascade, positive regulation of mitogen activated protein kinase kinase kinase cascade, positive regulation of mitogen-activated protein kinase cascade, positive regulation of mitogen-activated protein kinase kinase kinase cascade, stimulation of MAPK cascade, up regulation of MAPKKK cascade, up-regulation of MAPK cascade, up-regulation of MAPKKK cascade, upregulation of MAPK cascade, upregulation of MAPKKK cascade, activation of MAPK cascade, activation of MAPKKK cascade, stimulation of MAPKKK cascade Relationships: is a type of regulation of MAPK cascade [GO:0043408]; is_a positive regulation of intracellular signal transduction [GO:1902533]; positively regulates GO:0000165 Definition: Any process that activates or increases the frequency, rate or extent of signal transduction mediated by the MAPK cascade.